{
  "term_label": "polyadenylation-dependent ncRNA catabolic process",
  "gene": "UniProtKB:Q8NDF8",
  "gene_symbol": "TENT4B",
  "term_id": "GO:0043634",
  "gene_name": "Terminal nucleotidyltransferase 4B"
}